{
  "gene_name": "Immunoglobulin heavy variable 1-69-2",
  "gene": "UniProtKB:A0A0G2JMI3",
  "term_id": "UNKNOWN:0003",
  "term_label": "Unknown cellular component",
  "gene_symbol": "IGHV1-69-2"
}